positive regulation of endothelial cell development [GO:1901552] (biological process) References: PMID:19470579 Sources: GOC:TermGenie, GOC:pr Definition: Any process that activates or increases the frequency, rate or extent of endothelial cell development. Subtypes: GO:1903142 Also known as: up regulation of endothelial cell development, up-regulation of endothelial cell development, upregulation of endothelial cell development, activation of endothelial cell development Relationships: is a type of positive regulation of cell development [GO:0010720]; is a type of regulation of endothelial cell development [GO:1901550]; RO_0002213 GO:0001885